cyclin/CDK positive transcription elongation factor complex [GO:0008024] (CC) Also known as: positive transcription elongation factor complex b Definition: A transcription elongation factor complex that facilitates the transition from abortive to productive elongation by phosphorylating the CTD domain of the large subunit of DNA-directed RNA polymerase II, holoenzyme. Contains a cyclin and a cyclin-dependent protein kinase catalytic subunit. Relationships: is a type of GO:0008023; is a type of nuclear cyclin-dependent protein kinase holoenzyme complex [GO:0019908]; is a type of carboxy-terminal domain protein kinase complex [GO:0032806] References: PMID:10766736, PMID:16721054, PMID:17079683, PMID:19328067, PMID:7759473 Sources: GOC:bhm, GOC:vw Subtypes: P-TEFb complex [GO:0070691], GO:0070692 Note: See also the cellular component terms 'cyclin-dependent protein kinase activating kinase holoenzyme complex ; GO:0019907' and 'DNA-directed RNA polymerase II, holoenzyme ; GO:0016591'.